{
  "gene": "UniProtKB:Q9Y5W8",
  "term_id": "GO:0005769",
  "gene_name": "Sorting nexin-13",
  "term_label": "early endosome",
  "gene_symbol": "SNX13"
}